{
  "term_label": "membrane",
  "gene_name": "Synapse differentiation-inducing gene protein 1-like",
  "term_id": "GO:0016020",
  "gene_symbol": "SYNDIG1L",
  "gene": "UniProtKB:A6NDD5"
}